lactose transmembrane transporter activity [GO:0015155] (molecular function) Definition: Enables the transfer of lactose from one side of a membrane to the other. Lactose is a disaccharide 4-O-beta-D-galactopyranosyl-D-glucose, and constitutes roughly 5% of the milk in almost all mammals. Sources: GOC:mtg_transport, ISBN:0198506732, ISBN:0815340729 Also known as: lactose permease activity, lactose/glucose efflux transporter activity Relationships: is a type of GO:0015154; is part of GO:0015767 Subtypes: lactose:proton symporter activity [GO:0015528], protein-N(PI)-phosphohistidine-lactose phosphotransferase system transporter activity [GO:0022869]